vitamin E metabolic process [GO:0042360] (biological process) Definition: The chemical reactions and pathways involving vitamin E, tocopherol, which includes a series of eight structurally similar compounds. Alpha-tocopherol is the most active form in humans and is a powerful biological antioxidant. Sources: GOC:jl, ISBN:0198506732 Relationships: is a type of GO:0008152 Also known as: tocopherol metabolic process, tocopherol metabolism, vitamin E metabolism, alpha-tocopherol metabolic process, alpha-tocopherol metabolism Subtypes: vitamin E biosynthetic process [GO:0010189]